{
  "gene_symbol": "FOXI2",
  "gene_name": "Forkhead box protein I2",
  "gene": "UniProtKB:Q6ZQN5",
  "term_id": "GO:0000981",
  "term_label": "DNA-binding transcription factor activity, RNA polymerase II-specific"
}